{
  "gene_symbol": "GRINA",
  "term_label": "endoplasmic reticulum",
  "term_id": "GO:0005783",
  "gene_name": "Protein lifeguard 1",
  "gene": "UniProtKB:Q7Z429"
}